regulation of jasmonic acid metabolic process [GO:0080140] (biological process) Definition: Any process that modulates the frequency, rate or extent of the chemical reactions and pathways involving jasmonic acid. Sources: GOC:dhl Subtypes: regulation of jasmonic acid biosynthetic process [GO:0080141] Relationships: is a type of regulation of fatty acid metabolic process [GO:0019217]; regulates jasmonic acid metabolic process [GO:0009694]